{
  "gene": "UniProtKB:A0A075B6W5",
  "term_label": "Unknown biological process",
  "term_id": "UNKNOWN:0002",
  "gene_name": "T cell receptor alpha variable 23_delta variable 6",
  "gene_symbol": "TRAV23DV6"
}